{
  "gene": "UniProtKB:Q15744",
  "term_id": "UNKNOWN:0003",
  "gene_name": "CCAAT_enhancer-binding protein epsilon",
  "term_label": "Unknown cellular component",
  "gene_symbol": "CEBPE"
}